{
  "gene": "UniProtKB:Q9H9R9",
  "gene_symbol": "DBNDD1",
  "gene_name": "Dysbindin domain-containing protein 1",
  "term_id": "UNKNOWN:0001",
  "term_label": "Unknown molecular function"
}